{
  "term_label": "Unknown biological process",
  "gene_symbol": "HSPG2",
  "gene_name": "Basement membrane-specific heparan sulfate proteoglycan core protein",
  "term_id": "UNKNOWN:0002",
  "gene": "UniProtKB:P98160"
}